{
  "term_label": "cytoplasm",
  "gene_symbol": "GSK3B",
  "gene_name": "Glycogen synthase kinase-3 beta",
  "gene": "UniProtKB:P49841",
  "term_id": "GO:0005737"
}